collagen anchoring fibril [GO:0098648] (cellular component) Definition: A specialised collagen fibril that functions as an anchor, binding to other collagen structures. References: PMID:19945621 Sources: GOC:dos Subtypes: GO:0098652 Relationships: is a type of complex of collagen trimers [GO:0098644]; is part of GO:0140086